{
  "term_label": "cytosol",
  "gene_name": "Proteasome subunit beta type-9",
  "gene_symbol": "PSMB9",
  "term_id": "GO:0005829",
  "gene": "UniProtKB:P28065"
}